{
  "term_id": "UNKNOWN:0001",
  "term_label": "Unknown molecular function",
  "gene": "UniProtKB:Q9UKU7",
  "gene_symbol": "ACAD8",
  "gene_name": "Isobutyryl-CoA dehydrogenase, mitochondrial"
}